{
  "gene_name": "Putative cytochrome c oxidase subunit 7A3, mitochondrial",
  "term_label": "protein-macromolecule adaptor activity",
  "term_id": "GO:0030674",
  "gene": "UniProtKB:O60397",
  "gene_symbol": "COX7A2P2"
}